isocitrate dehydrogenase [NAD(P)+] activity [GO:0004448] (molecular function) Also known as: isocitrate dehydrogenase activity, isocitric acid dehydrogenase activity, isocitric dehydrogenase activity, oxalosuccinate carboxylase activity, oxalosuccinate decarboxylase activity, oxalosuccinic decarboxylase activity, IDH activity, IDP activity Subtypes: isocitrate dehydrogenase (NAD+) activity [GO:0004449], GO:0004450 Definition: Catalysis of the reaction: isocitrate + NAD(P)+ = 2-oxoglutarate + CO2 + NAD(P)H. Relationships: is a type of GO:0016616 Sources: GOC:curators